{
  "term_id": "UNKNOWN:0001",
  "gene": "UniProtKB:Q7Z3D4",
  "term_label": "Unknown molecular function",
  "gene_symbol": "LYSMD3",
  "gene_name": "LysM and putative peptidoglycan-binding domain-containing protein 3"
}